{
  "gene_symbol": "GAGE2A",
  "term_label": "Unknown molecular function",
  "gene_name": "G antigen 2A",
  "gene": "UniProtKB:Q6NT46",
  "term_id": "UNKNOWN:0001"
}